{
  "term_label": "Unknown molecular function",
  "gene": "UniProtKB:A0A5F9ZHS0",
  "gene_symbol": "A0A5F9ZHS0",
  "term_id": "UNKNOWN:0001",
  "gene_name": "Uncharacterized protein"
}